{
  "gene": "UniProtKB:P19367",
  "gene_name": "Hexokinase-1",
  "term_label": "mitochondrion",
  "term_id": "GO:0005739",
  "gene_symbol": "HK1"
}